{
  "gene_name": "Long-chain-fatty-acid--CoA ligase 1",
  "gene_symbol": "ACSL1",
  "term_id": "GO:0005783",
  "term_label": "endoplasmic reticulum",
  "gene": "UniProtKB:P33121"
}